{
  "term_id": "GO:0005886",
  "gene_symbol": "ANXA3",
  "gene": "UniProtKB:P12429",
  "term_label": "plasma membrane",
  "gene_name": "Annexin A3"
}